4-acetamidobutyryl-CoA deacetylase activity [GO:0047574] (molecular function) Definition: Catalysis of the reaction: 4-acetamidobutanoyl-CoA + H2O = 4-aminobutanoyl-CoA + acetate. Also known as: 4-acetamidobutanoyl-CoA amidohydrolase activity, aminobutyryl-CoA thiolesterase activity, deacetylase-thiolesterase activity Relationships: is a type of GO:0016811; is a type of GO:0019213 Sources: EC:3.5.1.51, RHEA:22928